maintenance of mitotic sister chromatid cohesion, telomeric [GO:0099403] (biological process) Definition: The process in which the association between sister chromatids of a replicated chromosome along the length of the telomeric region is maintained as chromosomes condense, attach to the spindle in a bipolar orientation, and congress to the metaphase plate during a mitotic cell cycle. References: PMID:26373281 Sources: GOC:BHF, GOC:BHF_telomere, GOC:dos, GOC:rph Regulation: regulated by regulation of maintenance of mitotic sister chromatid cohesion, telomeric [GO:1904907]; negatively regulated by GO:1904908; positively regulated by GO:1904909 Relationships: is a type of maintenance of mitotic sister chromatid cohesion [GO:0034088]; BFO_0000050 mitotic sister chromatid cohesion, telomeric [GO:0099404] Also known as: maintenance of mitotic sister chromatin cohesion at telomere, maintenance of sister chromatin cohesion at telomere at mitosis, maintenance of telomeric mitotic sister chromatin cohesion